{
  "gene_symbol": "A0A8I5KPI3",
  "gene_name": "Uncharacterized protein",
  "gene": "UniProtKB:A0A8I5KPI3",
  "term_label": "Unknown cellular component",
  "term_id": "UNKNOWN:0003"
}